{
  "term_label": "Unknown molecular function",
  "gene_symbol": "O00370",
  "gene_name": "LINE-1 retrotransposable element ORF2 protein",
  "gene": "UniProtKB:O00370",
  "term_id": "UNKNOWN:0001"
}